FFAT motif binding [GO:0033149] (molecular function) References: PMID:12727870, PMID:15455074, PMID:16004875 Definition: Binding to a FFAT motif, a short motif containing diphenylalanine in an acidic tract that targets proteins to the cytosolic surface of the ER and to the nuclear membrane by binding directly to members of the VAP (VAMP-associated protein) protein family. Relationships: is a type of protein domain specific binding [GO:0019904]